{
  "term_id": "GO:0005525",
  "gene": "UniProtKB:Q8IXI1",
  "gene_symbol": "RHOT2",
  "term_label": "GTP binding",
  "gene_name": "Mitochondrial Rho GTPase 2"
}